detection of nematode [GO:0009600] (biological process) Relationships: is a type of detection of other organism [GO:0098543] Also known as: perception of nematode Definition: The series of events in which a stimulus from a nematode is received and converted into a molecular signal. Sources: GOC:hb